{
  "term_id": "GO:0070652",
  "term_label": "HAUS complex",
  "gene_symbol": "HAUS5",
  "gene": "UniProtKB:O94927",
  "gene_name": "HAUS augmin-like complex subunit 5"
}